{
  "gene_symbol": "MDH1B",
  "gene_name": "Putative malate dehydrogenase 1B",
  "term_label": "malate metabolic process",
  "gene": "UniProtKB:Q5I0G3",
  "term_id": "GO:0006108"
}